Swi5-Sfr1 complex binding [GO:1905334] (molecular function) Definition: Binding to a Swi5-Sfr1 complex. References: PMID:16921379 Sources: GOC:TermGenie Relationships: is a type of protein-containing complex binding [GO:0044877] Also known as: Sae3-Mei5 complex binding